{
  "term_label": "unfolded protein binding",
  "gene_symbol": "CCT7",
  "term_id": "GO:0051082",
  "gene": "UniProtKB:Q99832",
  "gene_name": "T-complex protein 1 subunit eta"
}